{
  "term_label": "calmodulin binding",
  "gene_name": "Intermediate conductance calcium-activated potassium channel protein 4",
  "gene": "UniProtKB:O15554",
  "term_id": "GO:0005516",
  "gene_symbol": "KCNN4"
}